{
  "term_label": "delayed rectifier potassium channel activity",
  "gene": "UniProtKB:P17658",
  "gene_name": "Potassium voltage-gated channel subfamily A member 6",
  "gene_symbol": "KCNA6",
  "term_id": "GO:0005251"
}